{
  "term_id": "GO:0005546",
  "term_label": "phosphatidylinositol-4,5-bisphosphate binding",
  "gene_name": "Protein flightless-1 homolog",
  "gene_symbol": "FLII",
  "gene": "UniProtKB:Q13045"
}